ferrichrome import into cell [GO:0042928] (biological process) Also known as: ferrichrome transport Definition: A process in which ferrichrome is transported into the cell by specific cell surface receptors. Ferrichromes are any of a group of growth-promoting Fe(III) chelates formed by various genera of microfungi. They are homodetic cyclic hexapeptides made up of a tripeptide of glycine (or other small neutral amino acids) and a tripeptide of an N'acyl-N4-hydroxy-L-ornithine. Relationships: is a type of ferric-hydroxamate import into cell [GO:0015687]; is a type of amide transport [GO:0042886] References: PMID:23192658 Sources: GOC:jl, ISBN:0198506732